regulation of centrosome cycle [GO:0046605] (biological process) Definition: Any process that modulates the frequency, rate or extent of the centrosome cycle, the processes of centrosome duplication and separation. Sources: GOC:ai Relationships: is a type of regulation of cell cycle process [GO:0010564]; is a type of GO:0032886; is a type of regulation of cellular component organization [GO:0051128]; regulates centrosome cycle [GO:0007098] Subtypes: regulation of centrosome duplication [GO:0010824], negative regulation of centrosome cycle [GO:0046606], GO:0046607